{
  "term_id": "GO:0015693",
  "gene": "UniProtKB:Q0D2K0",
  "gene_symbol": "NIPAL4",
  "gene_name": "Magnesium transporter NIPA4",
  "term_label": "magnesium ion transport"
}